{
  "term_label": "cytoplasm",
  "gene": "UniProtKB:Q9UHH9",
  "gene_symbol": "IP6K2",
  "gene_name": "Inositol hexakisphosphate kinase 2",
  "term_id": "GO:0005737"
}